alpha-linked polysaccharide catabolism to maltopentaose [GO:0052787] (biological process) Definition: The breakdown of large alpha-linked polysaccharides by hydrolysis of (1->4)-alpha-D-glucosidic linkages to yield maltopentaose. References: PMID:7511484, PMID:9406414 Sources: GOC:mengo_curators Relationships: is a type of polysaccharide catabolic process [GO:0000272] Also known as: alpha-amylase-mediated polysaccharide catabolism, producing maltopentaose, maltopentaose-forming alpha-amylase activity